regulation of protein localization to cell division site involved in cell separation after cytokinesis [GO:1905391] (biological process) Definition: Any regulation of protein localization to cell division site that is involved in cell separation after cytokinesis. References: PMID:25411334 Sources: GOC:TermGenie, GO_REF:0000060 Also known as: regulation of protein localisation to cell division site involved in cell separation after cytokinesis, regulation of protein localisation to cell division site involved in cell separation following cytokinesis, regulation of protein localisation to cell division site involved in mitotic cytokinetic cell separation, regulation of protein localisation to cell division site involved in cytokinetic cell separation Relationships: is a type of regulation of protein localization to cell division site [GO:1901900]; BFO_0000050 GO:0000920